salicylic acid binding [GO:1901149] (molecular function) Definition: Binding to salicylic acid. Relationships: is a type of monocarboxylic acid binding [GO:0033293] References: PMID:22699612 Sources: GOC:TermGenie Also known as: salicylic acid receptor